{
  "gene_symbol": "PRKAR2B",
  "gene": "UniProtKB:P31323",
  "gene_name": "cAMP-dependent protein kinase type II-beta regulatory subunit",
  "term_id": "GO:0007189",
  "term_label": "adenylate cyclase-activating G protein-coupled receptor signaling pathway"
}